{
  "gene_symbol": "MGC35212",
  "gene_name": "Cell division control protein 24 OB domain-containing protein",
  "term_label": "Unknown cellular component",
  "gene": "UniProtKB:H3BU10",
  "term_id": "UNKNOWN:0003"
}